{
  "gene_name": "Interleukin-1 receptor-like 1",
  "gene_symbol": "IL1RL1",
  "term_id": "GO:0009986",
  "gene": "UniProtKB:Q01638",
  "term_label": "cell surface"
}